{
  "gene_symbol": "MAL",
  "term_label": "structural constituent of myelin sheath",
  "term_id": "GO:0019911",
  "gene_name": "Myelin and lymphocyte protein",
  "gene": "UniProtKB:P21145"
}